{
  "term_id": "UNKNOWN:0001",
  "term_label": "Unknown molecular function",
  "gene_symbol": "ZNF185",
  "gene_name": "Zinc finger protein 185",
  "gene": "UniProtKB:O15231"
}